{
  "term_id": "GO:0005829",
  "term_label": "cytosol",
  "gene_symbol": "GUK1",
  "gene_name": "Guanylate kinase",
  "gene": "UniProtKB:Q16774"
}